{
  "term_label": "Unknown biological process",
  "gene_symbol": "KRTAP1-4",
  "term_id": "UNKNOWN:0002",
  "gene": "UniProtKB:P0C5Y4",
  "gene_name": "Keratin-associated protein 1-4"
}